G-protein gated monoatomic cation channel activity [GO:0099100] (molecular function) Definition: A cation channel activity that is gated by binding of a G-protein beta-gamma dimer. Sources: GOC:dos Also known as: G-protein gated cation channel activity Relationships: is a type of G-protein gated monoatomic ion channel activity [GO:0099099]